{
  "gene_symbol": "OR8B3",
  "term_id": "UNKNOWN:0003",
  "gene": "UniProtKB:Q8NGG8",
  "term_label": "Unknown cellular component",
  "gene_name": "Olfactory receptor 8B3"
}